{
  "gene_name": "Hepatitis A virus cellular receptor 2",
  "term_id": "UNKNOWN:0001",
  "gene": "UniProtKB:Q8TDQ0",
  "gene_symbol": "HAVCR2",
  "term_label": "Unknown molecular function"
}